{
  "term_id": "GO:0005579",
  "gene_name": "Complement component C8 alpha chain",
  "gene_symbol": "C8A",
  "gene": "UniProtKB:P07357",
  "term_label": "membrane attack complex"
}